floral whorl morphogenesis [GO:0048457] (biological process) Sources: GOC:PO_curators, GOC:go_curators, PO:0025023 Definition: The process in which the anatomical structures of the floral whorl are generated and organized. Relationships: is a type of developmental process involved in reproduction [GO:0003006]; is a type of post-embryonic plant morphogenesis [GO:0090698]; is part of GO:0048438; is part of flower morphogenesis [GO:0048439]